{
  "gene_name": "Probable arginine--tRNA ligase, mitochondrial",
  "gene": "UniProtKB:Q5T160",
  "term_id": "GO:0032543",
  "term_label": "mitochondrial translation",
  "gene_symbol": "RARS2"
}